{
  "term_id": "GO:0007409",
  "gene": "UniProtKB:Q8IUH5",
  "gene_name": "Palmitoyltransferase ZDHHC17",
  "gene_symbol": "ZDHHC17",
  "term_label": "axonogenesis"
}